glycine secretion [GO:0061536] (BP) Definition: The controlled release of glycine by a cell. Sources: GOC:dph Relationships: is a type of glycine transport [GO:0015816]; is a type of secretion by cell [GO:0032940] Subtypes: GO:0061537